UV-damage excision repair [GO:0070914] (biological process) Definition: A DNA repair process that is initiated by an endonuclease that introduces a single-strand incision immediately 5' of a UV-induced damage site. UV-damage excision repair acts on both cyclobutane pyrimidine dimers (CPDs) and pyrimidine-pyrimidone 6-4 photoproducts (6-4PPs). Also known as: UV-damaged DNA endonuclease-dependent excision repair, UVDE-dependent excision repair, UVER, AER, alternative excision repair References: PMID:9619100 Sources: GOC:mah Relationships: is a type of DNA repair [GO:0006281]; is a type of cellular response to UV [GO:0034644]